{
  "term_id": "GO:0006955",
  "gene": "UniProtKB:A0A075B6K2",
  "term_label": "immune response",
  "gene_name": "Immunoglobulin lambda variable 3-12",
  "gene_symbol": "IGLV3-12"
}